plasma membrane raft [GO:0044853] (cellular component) Sources: GOC:jl Subtypes: caveola [GO:0005901], eisosome membrane domain/MCC [GO:0090512] Relationships: is a type of membrane raft [GO:0045121]; is a type of plasma membrane region [GO:0098590] Definition: A membrane raft that is part of the plasma membrane.